{
  "gene_name": "Lysosome membrane protein 2",
  "term_label": "scavenger receptor activity",
  "gene": "UniProtKB:Q14108",
  "gene_symbol": "SCARB2",
  "term_id": "GO:0005044"
}